sn-glycerol 3-phosphatase activity [GO:0043136] (MF) Definition: Catalysis of the reaction: H2O + sn-glycerol 3-phosphate = glycerol + phosphate. Sources: RHEA:66372 Relationships: is a type of phosphatase activity [GO:0016791] Also known as: glycerol-1-phosphatase activity, glycerol-3-phosphatase activity